{
  "gene_symbol": "SSX2B",
  "term_label": "Unknown biological process",
  "term_id": "UNKNOWN:0002",
  "gene_name": "Protein SSX2",
  "gene": "UniProtKB:Q16385"
}